vasoconstriction [GO:0042310] (biological process) Relationships: is a type of blood vessel diameter maintenance [GO:0097746] Definition: A decrease in the diameter of blood vessels, especially arteries, due to constriction of smooth muscle cells that line the vessels, and usually causing an increase in blood pressure. Sources: GOC:pr, ISBN:0192800752 Also known as: negative regulation of blood vessel size Regulation: regulated by regulation of vasoconstriction [GO:0019229]; negatively regulated by GO:0045906; positively regulated by positive regulation of vasoconstriction [GO:0045907] Subtypes: GO:0001987, GO:0001994, angiotensin-mediated vasoconstriction involved in regulation of systemic arterial blood pressure [GO:0001998], GO:0002006, GO:0002012, vasoconstriction of artery involved in ischemic response to lowering of systemic arterial blood pressure [GO:0002014], vascular associated smooth muscle contraction [GO:0014829]